Gi/o-coupled serotonin receptor activity [GO:0001586] (molecular function) Definition: Combining with serotonin and transmitting the signal across the membrane by activation of the Gi/o subunit of an associated cytoplasmic heterotrimeric G protein complex. The Gi/o subunit subsequently inhibits adenylate cyclase and results in a decrease in cyclic AMP (cAMP) levels. References: PMID:18571247 Sources: GOC:mah Also known as: 5-HT1 receptor activity, serotonin receptor activity, coupled via Gi/o Relationships: is a type of G protein-coupled serotonin receptor activity [GO:0004993]